interleukin-12 complex [GO:0043514] (cellular component) Note: Note that this heterodimeric cytokine utilizes the IL-12p35 subunit as its alpha chain, which is also used by IL-35 as its alpha chain, and utilizes the IL-12p40 subunit as its beta chain, which is also used by IL-23 as its beta chain. References: PMID:12948519, PMID:1381512 Sources: GOC:add, GOC:ebc, GOC:mah Also known as: IL-12 complex, IL12A, IL12B, p35, p40 Definition: A protein complex that is composed of an interleukin-12 alpha (p35, product of the IL12A gene) and an interleukin-12 beta subunit (p40, product of the IL12B gene) and is secreted into the extracellular space. Relationships: is a type of GO:0032991; BFO_0000050 GO:0005615